negative regulation of termination of RNA polymerase II transcription, poly(A)-coupled [GO:2000805] (biological process) Sources: GOC:obol Relationships: is a type of negative regulation of termination of RNA polymerase II transcription [GO:0120191]; is a type of regulation of termination of RNA polymerase II transcription, poly(A)-coupled [GO:2000804]; RO_0002212 termination of RNA polymerase II transcription, poly(A)-coupled [GO:0030846] Also known as: negative regulation of termination of RNA polymerase II transcription, polyadenylation-coupled, negative regulation of transcription termination from Pol II promoter, RNA polymerase(A) coupled, negative regulation of transcription termination from Pol II promoter, poly(A) coupled Definition: Any process that stops, prevents or reduces the frequency, rate or extent of termination of RNA polymerase II transcription, poly(A)-coupled.